{
  "gene": "UniProtKB:Q5JU85",
  "term_label": "regulation of postsynaptic neurotransmitter receptor internalization",
  "gene_symbol": "IQSEC2",
  "term_id": "GO:0099149",
  "gene_name": "IQ motif and SEC7 domain-containing protein 2"
}